{
  "gene": "UniProtKB:O75821",
  "term_label": "translational initiation",
  "gene_symbol": "EIF3G",
  "term_id": "GO:0006413",
  "gene_name": "Eukaryotic translation initiation factor 3 subunit G"
}